{
  "gene_name": "T cell receptor beta joining 2-2",
  "gene": "UniProtKB:A0A0A0MT94",
  "term_id": "UNKNOWN:0003",
  "term_label": "Unknown cellular component",
  "gene_symbol": "TRBJ2-2"
}